{
  "term_id": "UNKNOWN:0002",
  "gene_symbol": "AASDH",
  "gene": "UniProtKB:Q4L235",
  "gene_name": "Beta-alanine-activating enzyme",
  "term_label": "Unknown biological process"
}